{
  "term_id": "GO:0072380",
  "gene_name": "Small glutamine-rich tetratricopeptide repeat-containing protein alpha",
  "gene_symbol": "SGTA",
  "term_label": "TRC complex",
  "gene": "UniProtKB:O43765"
}